plasmid maintenance [GO:0006276] (biological process) Definition: The maintenance of the integrity of extrachromosomal plasmid DNA; includes processes that ensure plasmids are retained in the daughter cells after cell division. Sources: GOC:ai Subtypes: plasmid partitioning [GO:0030541], plasmid copy number maintenance [GO:0060908] Relationships: is a type of GO:0009987